regulation of hepatic stellate cell proliferation [GO:1904897] (biological process) Definition: Any process that modulates the frequency, rate or extent of hepatic stellate cell proliferation. References: PMID:15358192 Sources: GOC:TermGenie, GO_REF:0000058 Also known as: regulation of Ito cell proliferation, regulation of hepatic perisinusoidal cell proliferation, regulation of perisinusoidal cell proliferation Relationships: is_a regulation of fibroblast proliferation [GO:0048145]; RO_0002211 hepatic stellate cell proliferation [GO:1990922] Subtypes: GO:1904898, positive regulation of hepatic stellate cell proliferation [GO:1904899]